{
  "term_label": "positive regulation of canonical Wnt signaling pathway",
  "term_id": "GO:0090263",
  "gene_symbol": "NEK4",
  "gene_name": "Serine_threonine-protein kinase Nek4",
  "gene": "UniProtKB:P51957"
}